sorocarp spore cell differentiation [GO:0044671] (biological process) Definition: The process in which a relatively unspecialized cell acquires specialized features of a sorocarp spore cell, a cell of the sorocarp sorus. A sorocarp is the fruiting body characteristic of certain cellular slime moulds (e.g., Dictyosteliida) and consists of both stalk and a sorus (spore mass). Sources: GOC:jl, GOC:rjd Relationships: is_a cell differentiation [GO:0030154]; is part of sorocarp sorus development [GO:0048837] Regulation: regulated by regulation of sorocarp spore cell differentiation [GO:1901261]; negatively regulated by GO:1901262; positively regulated by GO:1901263